{
  "gene_symbol": "TBC1D3L",
  "term_id": "UNKNOWN:0002",
  "gene_name": "TBC1 domain family member 3L",
  "term_label": "Unknown biological process",
  "gene": "UniProtKB:B9A6J9"
}